{
  "term_id": "GO:0007040",
  "gene_name": "Clavesin-2",
  "term_label": "lysosome organization",
  "gene_symbol": "CLVS2",
  "gene": "UniProtKB:Q5SYC1"
}